eosinophil activation [GO:0043307] (biological process) Definition: The change in morphology and behavior of a eosinophil resulting from exposure to a cytokine, chemokine, cellular ligand, or soluble factor. Sources: GOC:add, ISBN:0781735149 Relationships: is a type of granulocyte activation [GO:0036230] Subtypes: eosinophil activation involved in immune response [GO:0002278] Regulation: regulated by GO:1902566; negatively regulated by negative regulation of eosinophil activation [GO:1902567]; positively regulated by positive regulation of eosinophil activation [GO:1902568]